{
  "term_id": "UNKNOWN:0003",
  "gene_symbol": "DEFB118",
  "term_label": "Unknown cellular component",
  "gene": "UniProtKB:Q96PH6",
  "gene_name": "Defensin beta 118"
}